{
  "gene_symbol": "HSPA8",
  "term_id": "GO:0005634",
  "gene_name": "Heat shock cognate 71 kDa protein",
  "term_label": "nucleus",
  "gene": "UniProtKB:P11142"
}